{
  "term_id": "GO:0000981",
  "term_label": "DNA-binding transcription factor activity, RNA polymerase II-specific",
  "gene": "UniProtKB:Q9BYE0",
  "gene_symbol": "HES7",
  "gene_name": "Transcription factor HES-7"
}